{
  "gene_name": "Golgi-associated kinase 1A",
  "term_id": "UNKNOWN:0001",
  "term_label": "Unknown molecular function",
  "gene_symbol": "GASK1A",
  "gene": "UniProtKB:Q9UFP1"
}